maintenance of left/right asymmetry [GO:0061968] (biological process) Relationships: is_a pattern specification process [GO:0007389] References: PMID:18629866 Sources: GOC:BHF Definition: The organization process that preserves the asymmetry in an organism's body plan or part of an organism with respect to the left and right halves. Subtypes: maintenance of left sidedness [GO:0061969], maintenance of right sidedness [GO:0061970]